cGMP metabolic process [GO:0046068] (biological process) Definition: The chemical reactions and pathways involving cyclic GMP, guanosine 3',5'-phosphate. Sources: GOC:go_curators Also known as: cGMP metabolism Relationships: is a type of purine ribonucleotide metabolic process [GO:0009150]; is a type of GO:0052652 Subtypes: cGMP biosynthetic process [GO:0006182], cGMP catabolic process [GO:0046069]